embryonic shoot morphogenesis [GO:0010064] (biological process) Sources: GOC:tb Definition: The process in which the anatomical structures of embryonic shoot are generated and organized. Relationships: is a type of shoot system morphogenesis [GO:0010016]; is a type of GO:0048598 Also known as: primary shoot system morphogenesis